neuropeptide hormone activity [GO:0005184] (molecular function) Sources: GOC:mah Relationships: is a type of hormone activity [GO:0005179]; is a type of neuropeptide activity [GO:0160041] Subtypes: neurohypophyseal hormone activity [GO:0005185], eclosion hormone activity [GO:0008031], ecdysis-triggering hormone activity [GO:0008255], ecdysiostatic hormone activity [GO:0016087], prothoracicotrophic hormone activity [GO:0018445] Also known as: neurohormone Definition: The action characteristic of a neuropeptide hormone, any peptide hormone that acts in the central nervous system. A neuropeptide is any of several types of molecules found in brain tissue, composed of short chains of amino acids; they include endorphins, enkephalins, vasopressin, and others. They are often localized in axon terminals at synapses and are classified as putative neurotransmitters, although some are also hormones.